{
  "term_label": "chaperonin-containing T-complex",
  "gene_name": "T-complex protein 1 subunit delta",
  "term_id": "GO:0005832",
  "gene_symbol": "CCT4",
  "gene": "UniProtKB:P50991"
}